positive regulation of cellular extravasation [GO:0002693] (biological process) Relationships: is a type of positive regulation of leukocyte migration [GO:0002687]; is a type of regulation of cellular extravasation [GO:0002691]; positively regulates GO:0045123 Subtypes: positive regulation of neutrophil extravasation [GO:2000391], GO:2000409, positive regulation of eosinophil extravasation [GO:2000421], GO:2000439 Also known as: up regulation of cellular extravasation, up-regulation of cellular extravasation, upregulation of cellular extravasation, activation of cellular extravasation, stimulation of cellular extravasation Sources: GOC:add Definition: Any process that activates or increases the frequency, rate, or extent of cellular extravasation.